{
  "term_id": "GO:0005634",
  "term_label": "nucleus",
  "gene": "UniProtKB:P16403",
  "gene_symbol": "H1-2",
  "gene_name": "Histone H1.2"
}